{
  "term_id": "GO:0044548",
  "gene_name": "Protein S100-A11",
  "gene": "UniProtKB:P31949",
  "term_label": "S100 protein binding",
  "gene_symbol": "S100A11"
}